{
  "gene_symbol": "IFNGR2",
  "term_label": "cytokine-mediated signaling pathway",
  "term_id": "GO:0019221",
  "gene": "UniProtKB:P38484",
  "gene_name": "Interferon gamma receptor 2"
}